L-lysine catabolic process [GO:0019477] (biological process) Definition: The chemical reactions and pathways resulting in the breakdown of L-lysine, the L-enantiomer of (S)-2,6-diaminohexanoic acid. Subtypes: L-lysine catabolic process to glutarate, by acetylation [GO:0019473], L-lysine catabolic process to acetyl-CoA [GO:0019474], L-lysine fermentation [GO:0019475] Sources: GOC:go_curators, GOC:jsg, GOC:mah Relationships: is a type of lysine catabolic process [GO:0006554]; is a type of L-amino acid catabolic process [GO:0170035]; is a type of proteinogenic amino acid catabolic process [GO:0170040] Also known as: L-lysine breakdown, L-lysine catabolism, L-lysine degradation